regulation of appressorium formation [GO:0075017] (biological process) Also known as: regulation of appressorium formation on or near host Subtypes: GO:0075018, negative regulation of appressorium formation [GO:0075019] Sources: GOC:pamgo_curators Definition: Any process that modulates the frequency, rate or extent of symbiont appressorium formation. Relationships: is a type of regulation of anatomical structure morphogenesis [GO:0022603]; regulates GO:0075016